{
  "gene_symbol": "TM4SF1",
  "term_label": "Unknown molecular function",
  "term_id": "UNKNOWN:0001",
  "gene_name": "Transmembrane 4 L6 family member 1",
  "gene": "UniProtKB:P30408"
}